glucuronolactone reductase activity [GO:0047941] (molecular function) Sources: EC:1.1.1.20, RHEA:18925 Relationships: is a type of oxidoreductase activity, acting on the CH-OH group of donors, NAD or NADP as acceptor [GO:0016616] Definition: Catalysis of the reaction: L-gulono-1,4-lactone + NADP+ = D-glucurono-3,6-lactone + H+ + NADPH.